{
  "gene_name": "Interleukin-36 receptor antagonist protein",
  "gene_symbol": "IL36RN",
  "gene": "UniProtKB:Q9UBH0",
  "term_label": "cellular response to lipopolysaccharide",
  "term_id": "GO:0071222"
}